{
  "gene_name": "RecQ-like DNA helicase BLM",
  "gene": "UniProtKB:P54132",
  "gene_symbol": "BLM",
  "term_label": "DNA replication",
  "term_id": "GO:0006260"
}